positive regulation of extracellular matrix assembly [GO:1901203] (biological process) Sources: GOC:BHF, GOC:TermGenie Relationships: is a type of positive regulation of cellular component biogenesis [GO:0044089]; is a type of regulation of extracellular matrix assembly [GO:1901201]; is a type of GO:1903055; positively regulates extracellular matrix assembly [GO:0085029] Also known as: up regulation of extracellular matrix assembly, up-regulation of extracellular matrix assembly, upregulation of extracellular matrix assembly, activation of extracellular matrix assembly Definition: Any process that activates or increases the frequency, rate or extent of extracellular matrix assembly. Subtypes: positive regulation of basement membrane assembly involved in embryonic body morphogenesis [GO:1904261]